{
  "gene_symbol": "POLR3H",
  "term_label": "RNA polymerase III complex",
  "term_id": "GO:0005666",
  "gene": "UniProtKB:Q9Y535",
  "gene_name": "DNA-directed RNA polymerase III subunit RPC8"
}